{
  "term_label": "structural constituent of ribosome",
  "gene_name": "Small ribosomal subunit protein uS9",
  "gene_symbol": "RPS16",
  "term_id": "GO:0003735",
  "gene": "UniProtKB:P62249"
}